{
  "gene_symbol": "MARCHF8",
  "term_id": "GO:0061630",
  "gene": "UniProtKB:Q5T0T0",
  "gene_name": "E3 ubiquitin-protein ligase MARCHF8",
  "term_label": "ubiquitin protein ligase activity"
}